{
  "term_id": "GO:0005886",
  "gene": "UniProtKB:Q8IVW1",
  "term_label": "plasma membrane",
  "gene_symbol": "ARL17A",
  "gene_name": "ADP-ribosylation factor-like protein 17"
}